{
  "term_id": "GO:0006626",
  "gene": "UniProtKB:Q8TB36",
  "gene_name": "Ganglioside-induced differentiation-associated protein 1",
  "gene_symbol": "GDAP1",
  "term_label": "protein targeting to mitochondrion"
}